{
  "gene_symbol": "HBG2",
  "term_id": "GO:0020037",
  "gene_name": "Hemoglobin subunit gamma-2",
  "term_label": "heme binding",
  "gene": "UniProtKB:P69892"
}